{
  "gene_name": "Diacylglycerol kinase gamma",
  "term_id": "GO:0004143",
  "gene_symbol": "DGKG",
  "gene": "UniProtKB:P49619",
  "term_label": "ATP-dependent diacylglycerol kinase activity"
}